{
  "gene_name": "NADH-ubiquinone oxidoreductase chain 2",
  "gene": "UniProtKB:P03891",
  "gene_symbol": "MT-ND2",
  "term_label": "NADH dehydrogenase (ubiquinone) activity",
  "term_id": "GO:0008137"
}